{
  "gene_symbol": "MALT1",
  "term_label": "positive regulation of canonical NF-kappaB signal transduction",
  "gene_name": "Mucosa-associated lymphoid tissue lymphoma translocation protein 1",
  "term_id": "GO:0043123",
  "gene": "UniProtKB:Q9UDY8"
}